{
  "gene": "UniProtKB:Q9NS82",
  "term_label": "D-alanine transmembrane transport",
  "term_id": "GO:0042941",
  "gene_name": "Asc-type amino acid transporter 1",
  "gene_symbol": "SLC7A10"
}